{
  "term_label": "Unknown molecular function",
  "gene_name": "Motile sperm domain-containing protein 2",
  "gene": "UniProtKB:Q8NHP6",
  "term_id": "UNKNOWN:0001",
  "gene_symbol": "MOSPD2"
}